{
  "term_label": "Unknown cellular component",
  "gene_name": "Zinc finger and BTB domain-containing protein 11",
  "gene_symbol": "ZBTB11",
  "term_id": "UNKNOWN:0003",
  "gene": "UniProtKB:O95625"
}